{
  "gene": "UniProtKB:P01911",
  "term_label": "peptide antigen assembly with MHC class II protein complex",
  "gene_symbol": "HLA-DRB1",
  "term_id": "GO:0002503",
  "gene_name": "HLA class II histocompatibility antigen, DRB1 beta chain"
}